{
  "term_label": "actin filament polymerization",
  "term_id": "GO:0030041",
  "gene": "UniProtKB:Q9Y3C0",
  "gene_symbol": "WASHC3",
  "gene_name": "WASH complex subunit 3"
}